angiotensin receptor activity [GO:0001595] (molecular function) Subtypes: angiotensin type I receptor activity [GO:0001596], angiotensin type II receptor activity [GO:0004945] Relationships: is a type of G protein-coupled peptide receptor activity [GO:0008528]; is part of GO:0038166 Definition: Combining with angiotensin to initiate a change in cell activity. Sources: GOC:ai